{
  "gene_symbol": "CALML3",
  "term_label": "myelin sheath",
  "term_id": "GO:0043209",
  "gene": "UniProtKB:P27482",
  "gene_name": "Calmodulin-like protein 3"
}